{
  "gene_name": "Centromere protein J",
  "term_id": "GO:0005814",
  "gene": "UniProtKB:Q9HC77",
  "term_label": "centriole",
  "gene_symbol": "CENPJ"
}